{
  "gene": "UniProtKB:Q9H252",
  "gene_name": "Potassium voltage-gated channel subfamily H member 6",
  "gene_symbol": "KCNH6",
  "term_label": "plasma membrane",
  "term_id": "GO:0005886"
}